{
  "term_id": "GO:0007155",
  "term_label": "cell adhesion",
  "gene": "UniProtKB:O76027",
  "gene_symbol": "ANXA9",
  "gene_name": "Annexin A9"
}